rubredoxin-NAD(P)H reductase activity [GO:0015045] (MF) Subtypes: GO:0015044, rubredoxin-NADP+ reductase activity [GO:0015046] Also known as: NADPH:rubredoxin reductase activity, NAD(P)--rubredoxin oxidoreductase activity, NAD(P)H--rubredoxin oxidoreductase activity, dinucleotide phosphate reductase activity, rubredoxin--nicotinamide adenine activity, rubredoxin--nicotinamide adenine dinucleotide (phosphate) reductase activity, rubredoxin:NAD(P)+ oxidoreductase activity Relationships: is a type of oxidoreductase activity, acting on iron-sulfur proteins as donors, NAD or NADP as acceptor [GO:0016731] Definition: Catalysis of the reaction: reduced rubredoxin + NAD(P)+ = oxidized rubredoxin + NAD(P)H + H+. Sources: EC:1.18.1.4